{
  "gene_symbol": "IQSEC1",
  "gene_name": "IQ motif and SEC7 domain-containing protein 1",
  "term_id": "GO:0005085",
  "term_label": "guanyl-nucleotide exchange factor activity",
  "gene": "UniProtKB:Q6DN90"
}